{
  "gene_symbol": "KLF12",
  "gene_name": "Krueppel-like factor 12",
  "term_label": "regulation of transcription by RNA polymerase II",
  "gene": "UniProtKB:Q9Y4X4",
  "term_id": "GO:0006357"
}